ornithine N-benzoyltransferase activity [GO:0050156] (molecular function) Also known as: benzoyl-CoA:L-ornithine N-benzoyltransferase activity, ornithine N-acyltransferase activity Sources: EC:2.3.1.127, RHEA:16929 Definition: Catalysis of the reaction: L-ornithine + 2 benzoyl-CoA = N(2),N(5)-dibenzoyl-L-ornithine + 2 CoA + 2 H+. Relationships: is_a GO:0016747